laminin-1 complex [GO:0005606] (cellular component) Also known as: laminin-111 complex References: PMID:10842354 Sources: GOC:jl Relationships: is a type of GO:0043256 Definition: A laminin complex composed of alpha1, beta1 and gamma1 polypeptide chains.